{
  "gene_name": "Pro-neuregulin-3, membrane-bound isoform",
  "term_id": "GO:0045499",
  "gene_symbol": "NRG3",
  "term_label": "chemorepellent activity",
  "gene": "UniProtKB:P56975"
}